{
  "gene_symbol": "SPG11",
  "gene": "UniProtKB:Q96JI7",
  "term_label": "synapse",
  "term_id": "GO:0045202",
  "gene_name": "Spatacsin"
}